{
  "term_label": "Unknown molecular function",
  "gene_symbol": "CMC2",
  "term_id": "UNKNOWN:0001",
  "gene": "UniProtKB:Q9NRP2",
  "gene_name": "COX assembly mitochondrial protein 2 homolog"
}